{
  "gene_name": "Leucine-rich repeat-containing protein 28",
  "gene_symbol": "LRRC28",
  "gene": "UniProtKB:Q86X40",
  "term_label": "Unknown cellular component",
  "term_id": "UNKNOWN:0003"
}